apoptotic process involved in heart morphogenesis [GO:0003278] (biological process) Sources: GOC:mtg_apoptosis, GOC:mtg_heart Relationships: is a type of GO:0060561; is part of heart morphogenesis [GO:0003007] Definition: Any apoptotic process that contributes to the shaping of the heart. Subtypes: apoptotic process involved in outflow tract morphogenesis [GO:0003275], apoptotic process involved in heart valve morphogenesis [GO:0003276], apoptotic process involved in endocardial cushion morphogenesis [GO:0003277], GO:0003296 Also known as: apoptosis involved in heart morphogenesis